{
  "gene_symbol": "ADAM21",
  "gene_name": "Disintegrin and metalloproteinase domain-containing protein 21",
  "gene": "UniProtKB:Q9UKJ8",
  "term_id": "GO:0006508",
  "term_label": "proteolysis"
}